{
  "gene_name": "Transforming growth factor-beta receptor type 3-like protein",
  "gene": "UniProtKB:H3BV60",
  "term_id": "GO:0005114",
  "term_label": "type II transforming growth factor beta receptor binding",
  "gene_symbol": "TGFBR3L"
}